{
  "term_id": "GO:0005886",
  "gene": "UniProtKB:P13726",
  "term_label": "plasma membrane",
  "gene_symbol": "F3",
  "gene_name": "Tissue factor"
}